{
  "term_label": "Unknown biological process",
  "gene": "UniProtKB:A0A0J9YVS3",
  "gene_name": "Immunoglobulin heavy joining 4 (Fragment)",
  "term_id": "UNKNOWN:0002",
  "gene_symbol": "IGHJ4"
}